{
  "term_id": "GO:0120094",
  "gene_name": "Chromodomain Y-like protein",
  "term_label": "negative regulation of peptidyl-lysine crotonylation",
  "gene_symbol": "CDYL",
  "gene": "UniProtKB:Q9Y232"
}